methionine gamma-lyase activity [GO:0018826] (molecular function) Definition: Catalysis of the reaction: L-methionine = methanethiol + NH3 + 2-oxobutanoate. Sources: EC:4.4.1.11, RHEA:23800 Also known as: L-methioninase activity, L-methionine gamma-lyase activity, L-methionine methanethiol-lyase (deaminating), L-methionine methanethiol-lyase (deaminating; 2-oxobutanoate-forming), methioninase activity, methionine dethiomethylase activity, methionine lyase activity Relationships: is a type of carbon-sulfur lyase activity [GO:0016846]